{
  "term_label": "RNA polymerase II cis-regulatory region sequence-specific DNA binding",
  "term_id": "GO:0000978",
  "gene": "UniProtKB:Q86T24",
  "gene_symbol": "ZBTB33",
  "gene_name": "Transcriptional regulator Kaiso"
}